{
  "term_id": "GO:0050729",
  "gene_name": "SET domain-containing protein 4",
  "gene": "UniProtKB:Q9NVD3",
  "gene_symbol": "SETD4",
  "term_label": "positive regulation of inflammatory response"
}